positive regulation of fumonisin biosynthetic process [GO:1900685] (biological process) Relationships: is_a positive regulation of small molecule metabolic process [GO:0062013]; is a type of positive regulation of secondary metabolite biosynthetic process [GO:1900378]; is a type of regulation of fumonisin biosynthetic process [GO:1900683]; positively regulates fumonisin biosynthetic process [GO:1900541] Sources: GOC:TermGenie, GOC:di Also known as: activation of fumonisin anabolism, activation of fumonisin biosynthesis, activation of fumonisin formation, activation of fumonisin synthesis, positive regulation of fumonisin anabolism, positive regulation of fumonisin biosynthesis, positive regulation of fumonisin formation, positive regulation of fumonisin synthesis, up regulation of fumonisin anabolism, up regulation of fumonisin biosynthesis, up regulation of fumonisin biosynthetic process, up regulation of fumonisin formation, up regulation of fumonisin synthesis, up-regulation of fumonisin anabolism, up-regulation of fumonisin biosynthesis, up-regulation of fumonisin biosynthetic process, up-regulation of fumonisin formation, up-regulation of fumonisin synthesis, upregulation of fumonisin anabolism, upregulation of fumonisin biosynthesis, upregulation of fumonisin biosynthetic process, upregulation of fumonisin formation, upregulation of fumonisin synthesis, activation of fumonisin biosynthetic process Definition: Any process that activates or increases the frequency, rate or extent of fumonisin biosynthetic process.